{
  "term_label": "Unknown cellular component",
  "gene_symbol": "SCYGR3",
  "gene_name": "Small cysteine and glycine repeat-containing protein 3",
  "gene": "UniProtKB:A0A286YF60",
  "term_id": "UNKNOWN:0003"
}